{
  "term_id": "GO:2001240",
  "gene": "UniProtKB:O00167",
  "gene_symbol": "EYA2",
  "term_label": "negative regulation of extrinsic apoptotic signaling pathway in absence of ligand",
  "gene_name": "Eyes absent homolog 2"
}